23S rRNA (guanine(2445)-N(2))-methyltransferase activity [GO:0052915] (molecular function) Sources: EC:2.1.1.173 Definition: Catalysis of the reaction: S-adenosyl-L-methionine + guanosine(2445) in 23S rRNA = N(2)-methylguanosine(2445) in 23S rRNA + S-adenosyl-L-homocysteine. Relationships: is a type of rRNA (guanine-N2-)-methyltransferase activity [GO:0008990]